{
  "term_id": "GO:0050855",
  "term_label": "regulation of B cell receptor signaling pathway",
  "gene": "UniProtKB:P07948",
  "gene_name": "Tyrosine-protein kinase Lyn",
  "gene_symbol": "LYN"
}